intestinal folate absorption [GO:0098829] (biological process) Relationships: is_a intestinal absorption [GO:0050892] Definition: Uptake of folic into the blood by absorption from the small intestine. References: PMID:19762432 Sources: GOC:BHF, GOC:dos, GOC:hal